host cell chloroplast thylakoid membrane [GO:0033654] (cellular component) Relationships: is a type of host cell chloroplast part [GO:0033653]; is a type of host thylakoid membrane [GO:0044160] Definition: Any sac-like membranous structures (cisternae) in a chloroplast found in host cells, combined into stacks (grana) and present singly in the stroma (stroma thylakoids or frets) as interconnections between grana. The host is defined as the larger of the organisms involved in a symbiotic interaction. Sources: GOC:pamgo_curators